{
  "gene_name": "Ankyrin repeat and sterile alpha motif domain-containing protein 1B",
  "term_label": "regulation of synaptic plasticity by receptor localization to synapse",
  "gene_symbol": "ANKS1B",
  "gene": "UniProtKB:Q7Z6G8",
  "term_id": "GO:1900383"
}